{
  "gene_name": "Lysophosphatidylserine lipase ABHD12",
  "gene": "UniProtKB:Q8N2K0",
  "term_label": "phosphatidylcholine lysophospholipase activity",
  "term_id": "GO:0004622",
  "gene_symbol": "ABHD12"
}